{
  "gene_name": "Josephin-1",
  "term_label": "cysteine-type deubiquitinase activity",
  "gene": "UniProtKB:Q15040",
  "gene_symbol": "JOSD1",
  "term_id": "GO:0004843"
}